ionotropic glutamate receptor binding [GO:0035255] (molecular function) Sources: GOC:bf, ISBN:0198506732 Definition: Binding to an ionotropic glutamate receptor. Ionotropic glutamate receptors bind glutamate and exert an effect through the regulation of ion channels. Relationships: is a type of glutamate receptor binding [GO:0035254]